stamen formation [GO:0048455] (biological process) Definition: The process that contributes to the act of giving rise to the stamen. This process pertains to the initial formation of a structure from unspecified parts. Sources: GOC:jid Relationships: is a type of floral organ formation [GO:0048449]; is part of GO:0048448